response to hermaphrodite contact [GO:0034606] (biological process) Definition: The response by the male to a hermaphrodite after initial contact following mate finding. The male stops forward locomotion, presses the ventral side of his tail against his partner's body, and begins moving backward along the hermaphrodite. Male response behavior is initiated when sensory neurons located in the rays of his tail contact a potential mate. Relationships: is a type of male mating behavior [GO:0060179] References: PMID:18050467 Sources: WB_REF:WBPaper00002109